{
  "term_label": "chromatin binding",
  "gene_name": "Chromobox protein homolog 5",
  "term_id": "GO:0003682",
  "gene": "UniProtKB:P45973",
  "gene_symbol": "CBX5"
}